{
  "gene_symbol": "MAP6",
  "gene": "UniProtKB:Q96JE9",
  "gene_name": "Microtubule-associated protein 6",
  "term_id": "GO:0030424",
  "term_label": "axon"
}